{
  "gene": "UniProtKB:Q14155",
  "term_label": "lamellipodium assembly",
  "gene_symbol": "ARHGEF7",
  "gene_name": "Rho guanine nucleotide exchange factor 7",
  "term_id": "GO:0030032"
}